negative regulation of motor neuron migration [GO:1905484] (biological process) References: PMID:16516839 Sources: GOC:TermGenie, GO_REF:0000058 Subtypes: negative regulation of lateral motor column neuron migration [GO:1902077] Relationships: is a type of regulation of motor neuron migration [GO:1905483]; is a type of negative regulation of neuron migration [GO:2001223]; negatively regulates motor neuron migration [GO:0097475] Also known as: down regulation of motor neuron migration, down-regulation of motor neuron migration, downregulation of motor neuron migration, inhibition of motor neuron migration Definition: Any process that stops, prevents or reduces the frequency, rate or extent of motor neuron migration.